{
  "gene": "UniProtKB:Q14202",
  "gene_name": "Zinc finger MYM-type protein 3",
  "gene_symbol": "ZMYM3",
  "term_label": "Unknown cellular component",
  "term_id": "UNKNOWN:0003"
}